regulation of R8 cell differentiation [GO:0045679] (biological process) Sources: GOC:go_curators Subtypes: negative regulation of R8 cell differentiation [GO:0045680], positive regulation of R8 cell differentiation [GO:0045681] Definition: Any process that modulates the frequency, rate or extent of R8 differentiation. Relationships: is a type of GO:0110116; regulates R8 cell differentiation [GO:0045465]